{
  "gene": "UniProtKB:Q2KHT3",
  "gene_symbol": "CLEC16A",
  "term_id": "GO:0016197",
  "gene_name": "Protein CLEC16A",
  "term_label": "endosomal transport"
}